glycoprotein-N-acetylgalactosamine 3-beta-galactosyltransferase activity [GO:0016263] (molecular function) Definition: Catalysis of the addition of a galactosyl residue to a non-reducing O-linked N-acetylgalactosamine residue in an O-glycan. Relationships: is a type of beta-1,3-galactosyltransferase activity [GO:0048531]; is a type of catalytic activity, acting on a glycoprotein [GO:0140103] Sources: EC:2.4.1.122, GOC:ma Also known as: Core 1 GalT, UDP-galactose:glycoprotein-N-acetyl-D-galactosamine 3-beta-D-galactosyltransferase activity, UDPgalactose:glycoprotein-N-acetyl-D-galactosamine 3-beta-D-galactosyltransferase activity, uridine diphosphogalactose-mucin beta-(1->3)-galactosyltransferase activity